{
  "gene": "UniProtKB:Q68J44",
  "gene_symbol": "DUSP29",
  "term_id": "GO:0008138",
  "term_label": "protein tyrosine/serine/threonine phosphatase activity",
  "gene_name": "Dual specificity phosphatase 29"
}